histone H3R26 arginine deiminase activity [GO:0140798] (molecular function) References: PMID:15339660 Definition: Catalysis of the reaction: H2O + histone H3 L-arginyl (position 26)= histone H3 L-citrullyl (position 26) + NH4+, resulting in histone H3 citrullination at position 26. Also known as: H3-R26 citrullination, histone H3-R26 arginine deiminase activity, histone-arginine deiminase activity (H3-R26 specific) Note: Comment: Note that the residue position corresponds to the canonical human H3 histone (UniProtKB:P84243); this residue is conserved across all eukaryotes. Residue 1 is the first residue following removal of the initiating Methionine (Met). Note that each histone is encoded by multiple genes, and sequences may vary across different genes within an organism. The substrate for histone deiminase may be methyl-arginine, rather than arginine (see PMID:35197210 and PMID:16567635). Relationships: is a type of histone H3 arginine deiminase activity [GO:0141057]